neural fold bending [GO:0021503] (BP) Definition: The morphogenesis of the neural fold elevations that results in the movement of the tips of the elevations towards each other in order to fuse. Relationships: is a type of GO:0048598; is a type of morphogenesis of an epithelial fold [GO:0060571]; is part of neural fold formation [GO:0001842] References: PMID:15806586 Sources: GOC:cls, GOC:dgh, GOC:dph, GOC:jid, GO_REF:0000021